interleukin-13 binding [GO:0019973] (molecular function) Also known as: IL-13 binding Sources: GOC:jl Definition: Binding to interleukin-13. Relationships: is a type of cytokine binding [GO:0019955]